free fatty acid 2-hydroxylase activity [GO:0120520] (molecular function) Relationships: is a type of fatty acid 2-hydroxylase activity [GO:0080132] Sources: GOC:sjm, RHEA:38855 Definition: Catalysis of the reaction: a 1,2-saturated fatty acid + 2 Fe(II)-[cytochrome b5] + 2 H+ + O2 = a (R)-2-hydroxy fatty acid + 2 Fe(III)-[cytochrome b5] + H2O. Note that the substrate is a free fatty acid, not a fatty acyl chain within a sphingolipid.